{
  "term_label": "phosphatidylethanolamine binding",
  "term_id": "GO:0008429",
  "gene_symbol": "MAP1LC3C",
  "gene_name": "Microtubule-associated proteins 1A_1B light chain 3C",
  "gene": "UniProtKB:Q9BXW4"
}